{
  "gene_name": "Hepatic and glial cell adhesion molecule",
  "term_id": "GO:0006955",
  "gene": "UniProtKB:Q14CZ8",
  "gene_symbol": "HEPACAM",
  "term_label": "immune response"
}